response to blue light [GO:0009637] (biological process) Sources: GOC:ai, GOC:mtg_far_red Relationships: is a type of response to light stimulus [GO:0009416] Definition: Any process that results in a change in state or activity of a cell or an organism (in terms of movement, secretion, enzyme production, gene expression, etc.) as a result of a blue light stimulus. Blue light is electromagnetic radiation with a wavelength of between 440 and 500nm. Also known as: blue light response, blue-light response, response to blue light stimulus Subtypes: phototropism [GO:0009638], response to photoperiod, blue light [GO:0009906], response to low fluence blue light stimulus by blue low-fluence system [GO:0010244], response to high fluence blue light stimulus by blue high-fluence system [GO:0055121], cellular response to blue light [GO:0071483]